{
  "term_id": "UNKNOWN:0001",
  "gene": "UniProtKB:B3EWG6",
  "gene_symbol": "FAM25G",
  "term_label": "Unknown molecular function",
  "gene_name": "Protein FAM25G"
}